transcription factor TFIIIB complex assembly [GO:0070217] (biological process) Also known as: TFIIIB assembly Sources: GOC:mah Relationships: is a type of protein-containing complex assembly [GO:0065003] Definition: The aggregation, arrangement and bonding together of a set of components to form a transcription factor TFIIIB complex.